{
  "term_id": "UNKNOWN:0003",
  "gene_name": "Proline-rich protein 35",
  "gene": "UniProtKB:P0CG20",
  "term_label": "Unknown cellular component",
  "gene_symbol": "PRR35"
}